{
  "gene_symbol": "EDA",
  "term_id": "GO:0043123",
  "gene_name": "Ectodysplasin-A",
  "gene": "UniProtKB:Q92838",
  "term_label": "positive regulation of canonical NF-kappaB signal transduction"
}